postsynaptic endocytic zone cytoplasmic component [GO:0099631] (cellular component) Definition: The cytoplasmic component of the postsynaptic endocytic zone. Relationships: is a type of cell cortex region [GO:0099738]; is part of postsynaptic endocytic zone [GO:0098843] Sources: GOC:dos